{
  "gene": "UniProtKB:Q6EMB2",
  "term_id": "GO:0015631",
  "gene_symbol": "TTLL5",
  "term_label": "tubulin binding",
  "gene_name": "Tubulin polyglutamylase TTLL5"
}